{
  "term_id": "GO:0000815",
  "gene_symbol": "CHMP4B",
  "term_label": "ESCRT III complex",
  "gene": "UniProtKB:Q9H444",
  "gene_name": "Charged multivesicular body protein 4b"
}